{
  "gene_symbol": "RGCC",
  "term_id": "GO:0005737",
  "gene": "UniProtKB:Q9H4X1",
  "gene_name": "Regulator of cell cycle RGCC",
  "term_label": "cytoplasm"
}